{
  "term_id": "UNKNOWN:0001",
  "term_label": "Unknown molecular function",
  "gene_name": "Inhibitor of growth protein 1",
  "gene_symbol": "ING1",
  "gene": "UniProtKB:Q9UK53"
}